phosphatidylcholine biosynthesis from choline and CDP-diacylglycerol [GO:0090639] (biological process) Relationships: is a type of phosphatidylcholine biosynthetic process [GO:0006656] Sources: MetaCyc:PWY-6826 Definition: The phosphatidylcholine biosynthetic process that involves a one-step direct condensation of choline with CDP-diacylglycerol to form phosphatidylcholine.